{
  "gene_symbol": "ZC3H7B",
  "gene": "UniProtKB:Q9UGR2",
  "term_label": "Unknown cellular component",
  "term_id": "UNKNOWN:0003",
  "gene_name": "Zinc finger CCCH domain-containing protein 7B"
}